{
  "term_id": "GO:0004984",
  "gene": "UniProtKB:P0DN80",
  "term_label": "olfactory receptor activity",
  "gene_name": "Olfactory receptor 5H8",
  "gene_symbol": "OR5H8"
}